{
  "gene_symbol": "FAM3A",
  "gene_name": "Protein FAM3A",
  "term_label": "cytokine activity",
  "term_id": "GO:0005125",
  "gene": "UniProtKB:P98173"
}